{
  "term_label": "DNA damage response",
  "gene_symbol": "PLK3",
  "gene_name": "Serine_threonine-protein kinase PLK3",
  "term_id": "GO:0006974",
  "gene": "UniProtKB:Q9H4B4"
}